DNA-directed DNA polymerase activity [GO:0003887] (molecular function) Also known as: duplicase, DNA polymerase I, DNA polymerase II, DNA polymerase III, DNA polymerase V activity, DNA polymerase alpha, DNA polymerase beta, DNA polymerase gamma, Klenow fragment, Taq DNA polymerase, Taq Pol I, Tca DNA polymerase, alpha DNA polymerase activity, beta DNA polymerase activity, delta DNA polymerase activity, deoxyribonucleic polymerase I, epsilon DNA polymerase activity, eta DNA polymerase activity, gamma DNA-directed DNA polymerase activity, iota DNA polymerase activity, kappa DNA polymerase activity, lambda DNA polymerase activity, mu DNA polymerase activity, nu DNA polymerase activity, sigma DNA polymerase activity, theta DNA polymerase activity, zeta DNA polymerase activity, DNA duplicase activity, DNA nucleotidyltransferase (DNA-directed) activity, DNA replicase activity, DNA-dependent DNA polymerase activity, deoxynucleoside-triphosphate:DNA deoxynucleotidyltransferase (DNA-directed) activity, deoxyribonucleic acid duplicase activity, deoxyribonucleic duplicase activity, sequenase Sources: EC:2.7.7.7, GOC:vw Regulation: positively regulated by positive regulation of DNA-directed DNA polymerase activity [GO:1900264] Relationships: is a type of GO:0034061 Definition: Catalysis of the reaction: deoxynucleoside triphosphate + DNA(n) = diphosphate + DNA(n+1); DNA-template-directed extension of the 3'-end of a DNA strand by one nucleotide at a time.